{
  "gene": "UniProtKB:Q969U7",
  "term_label": "cytosol",
  "gene_symbol": "PSMG2",
  "gene_name": "Proteasome assembly chaperone 2",
  "term_id": "GO:0005829"
}